{
  "term_id": "UNKNOWN:0001",
  "gene_name": "Condensin complex subunit 3",
  "gene": "UniProtKB:Q9BPX3",
  "gene_symbol": "NCAPG",
  "term_label": "Unknown molecular function"
}